{
  "gene_symbol": "RRAGB",
  "gene": "UniProtKB:Q5VZM2",
  "term_label": "nucleus",
  "term_id": "GO:0005634",
  "gene_name": "Ras-related GTP-binding protein B"
}